{
  "term_id": "GO:0005737",
  "gene": "UniProtKB:Q9UNH5",
  "gene_name": "Dual specificity protein phosphatase CDC14A",
  "gene_symbol": "CDC14A",
  "term_label": "cytoplasm"
}